negative regulation of hypoxia-inducible factor-1alpha signaling pathway [GO:1902072] (biological process) Definition: Any process that stops, prevents or reduces the frequency, rate or extent of hypoxia-inducible factor-1alpha signaling pathway. Sources: GOC:TermGenie, GOC:bf Also known as: down regulation of HIF1alpha pathway, down regulation of hypoxia-inducible factor-1alpha signaling pathway, down regulation of hypoxia-inducible factor-1alpha signalling pathway, down-regulation of HIF1alpha pathway, down-regulation of hypoxia-inducible factor-1alpha signaling pathway, down-regulation of hypoxia-inducible factor-1alpha signalling pathway, downregulation of HIF1alpha pathway, downregulation of hypoxia-inducible factor-1alpha signaling pathway, downregulation of hypoxia-inducible factor-1alpha signalling pathway, inhibition of HIF1alpha pathway, inhibition of hypoxia-inducible factor-1alpha signalling pathway, negative regulation of HIF1alpha pathway, negative regulation of hypoxia-inducible factor-1alpha signalling pathway, inhibition of hypoxia-inducible factor-1alpha signaling pathway Relationships: is a type of GO:1900038; is a type of regulation of hypoxia-inducible factor-1alpha signaling pathway [GO:1902071]; is_a GO:1902532; negatively regulates GO:0097411